{
  "gene": "UniProtKB:Q96BS2",
  "term_label": "nucleus",
  "gene_symbol": "TESC",
  "term_id": "GO:0005634",
  "gene_name": "Calcineurin B homologous protein 3"
}